{
  "gene_symbol": "OBSCN",
  "term_label": "M band",
  "gene_name": "Obscurin",
  "term_id": "GO:0031430",
  "gene": "UniProtKB:Q5VST9"
}